{
  "gene_symbol": "SLC47A2",
  "gene": "UniProtKB:Q86VL8",
  "gene_name": "Multidrug and toxin extrusion protein 2",
  "term_label": "membrane",
  "term_id": "GO:0016020"
}